{
  "gene_symbol": "MRPS31",
  "gene": "UniProtKB:Q92665",
  "term_label": "Unknown biological process",
  "term_id": "UNKNOWN:0002",
  "gene_name": "Small ribosomal subunit protein mS31"
}